positive regulation of stress-activated MAPK cascade [GO:0032874] (BP) Subtypes: positive regulation of cell integrity MAPK cascade [GO:1903139] Also known as: positive regulation of p38 MAPK signaling, positive regulation of p38 MAPK signalling, positive regulation of stress-activated MAPK signaling pathway, positive regulation of stress-activated MAPK signalling pathway, positive regulation of stress-activated MAPKKK cascade, positive regulation of stress-activated MAPKKK signaling pathway, positive regulation of stress-activated MAPKKK signalling pathway, up regulation of stress-activated MAPK cascade, up-regulation of stress-activated MAPK cascade, upregulation of stress-activated MAPK cascade, activation of stress-activated MAPK cascade, stimulation of stress-activated MAPK cascade Definition: Any process that activates or increases the frequency, rate or extent of signal transduction mediated by the stress-activated MAPK cascade. Relationships: is a type of regulation of stress-activated MAPK cascade [GO:0032872]; is a type of positive regulation of MAPK cascade [GO:0043410]; is a type of positive regulation of stress-activated protein kinase signaling cascade [GO:0070304]; positively regulates stress-activated MAPK cascade [GO:0051403] Sources: GOC:mah